{
  "term_label": "SNARE binding",
  "gene_symbol": "TSNARE1",
  "term_id": "GO:0000149",
  "gene_name": "t-SNARE domain-containing protein 1",
  "gene": "UniProtKB:Q96NA8"
}